dendrite development by retrograde extension [GO:0003390] (biological process) Relationships: is a type of retrograde extension [GO:0003389]; is a type of GO:0016358 Subtypes: GO:0003391 Sources: GOC:ascb_2009, GOC:dph, GOC:tb Also known as: dendrite retrograde extension Definition: The progression of a dendrite over time by the attachment of a part of the neuron to an anchor and the subsequent migration of the cell body away from the anchor point.